{
  "gene_name": "Mediator of RNA polymerase II transcription subunit 14",
  "gene_symbol": "MED14",
  "term_id": "GO:0006357",
  "gene": "UniProtKB:O60244",
  "term_label": "regulation of transcription by RNA polymerase II"
}